platelet maturation [GO:0036345] (biological process) Definition: A developmental process, independent of morphogenetic (shape) change, that is required for a platelet to attain its fully functional state. A platelet is a non-nucleated disk-shaped cell formed by extrusion from megakaryocytes, found in the blood of all mammals, and mainly involved in blood coagulation. Relationships: is a type of cell maturation [GO:0048469] Sources: CL:0000233, GOC:BHF, GOC:vk